{
  "term_id": "UNKNOWN:0003",
  "gene_symbol": "ZNF382",
  "gene_name": "Zinc finger protein 382",
  "term_label": "Unknown cellular component",
  "gene": "UniProtKB:Q96SR6"
}